{
  "gene_symbol": "CALHM1",
  "term_id": "GO:0005886",
  "gene": "UniProtKB:Q8IU99",
  "gene_name": "Calcium homeostasis modulator protein 1",
  "term_label": "plasma membrane"
}